{
  "gene": "UniProtKB:Q2M3C7",
  "gene_name": "A-kinase anchor protein SPHKAP",
  "gene_symbol": "SPHKAP",
  "term_label": "protein kinase A binding",
  "term_id": "GO:0051018"
}